{
  "gene": "UniProtKB:Q9Y6Q2",
  "gene_symbol": "STON1",
  "gene_name": "Stonin-1",
  "term_id": "GO:0005829",
  "term_label": "cytosol"
}